negative regulation of progesterone biosynthetic process [GO:2000183] (biological process) Definition: Any process that stops, prevents, or reduces the frequency, rate or extent of progesterone biosynthetic process. Subtypes: GO:0061363 Relationships: is a type of negative regulation of steroid biosynthetic process [GO:0010894]; is a type of negative regulation of hormone biosynthetic process [GO:0032353]; is a type of negative regulation of small molecule metabolic process [GO:0062014]; is a type of GO:2000182; negatively regulates progesterone biosynthetic process [GO:0006701] Also known as: negative regulation of progesterone anabolism, negative regulation of progesterone biosynthesis, negative regulation of progesterone formation, negative regulation of progesterone synthesis Sources: GOC:dph